{
  "term_id": "GO:0098609",
  "gene_name": "Plakophilin-1",
  "term_label": "cell-cell adhesion",
  "gene": "UniProtKB:Q13835",
  "gene_symbol": "PKP1"
}